{
  "term_id": "GO:0032870",
  "term_label": "cellular response to hormone stimulus",
  "gene": "UniProtKB:O60896",
  "gene_symbol": "RAMP3",
  "gene_name": "Receptor activity-modifying protein 3"
}